{
  "gene": "UniProtKB:Q9BQP9",
  "term_id": "UNKNOWN:0001",
  "gene_name": "BPI fold-containing family A member 3",
  "term_label": "Unknown molecular function",
  "gene_symbol": "BPIFA3"
}